{
  "gene": "UniProtKB:Q9UFC0",
  "gene_symbol": "LRWD1",
  "term_id": "GO:0071169",
  "gene_name": "Leucine-rich repeat and WD repeat-containing protein 1",
  "term_label": "establishment of protein localization to chromatin"
}